{
  "term_label": "mitochondrial translational elongation",
  "gene_symbol": "TUFM",
  "term_id": "GO:0070125",
  "gene": "UniProtKB:P49411",
  "gene_name": "Elongation factor Tu, mitochondrial"
}